{
  "gene_symbol": "SFR1",
  "term_label": "transcription coactivator activity",
  "gene_name": "Swi5-dependent recombination DNA repair protein 1 homolog",
  "gene": "UniProtKB:Q86XK3",
  "term_id": "GO:0003713"
}